prephenate dehydrogenase (NADP+) activity [GO:0004665] (molecular function) Relationships: is a type of oxidoreductase activity, acting on the CH-CH group of donors, NAD or NADP as acceptor [GO:0016628] Also known as: prephenate (nicotinamide adenine dinucleotide phosphate) dehydrogenase activity, prephenate:NADP+ oxidoreductase (decarboxylating) Sources: EC:1.3.1.13, RHEA:21640 Definition: Catalysis of the reaction: NADP+ + prephenate = (4-hydroxyphenyl)pyruvate + CO2 + NADPH.